{
  "gene_symbol": "GMPR",
  "term_id": "UNKNOWN:0003",
  "gene_name": "GMP reductase 1",
  "gene": "UniProtKB:P36959",
  "term_label": "Unknown cellular component"
}